{
  "term_label": "Unknown cellular component",
  "gene_symbol": "ASB9",
  "gene": "UniProtKB:Q96DX5",
  "term_id": "UNKNOWN:0003",
  "gene_name": "Ankyrin repeat and SOCS box protein 9"
}